low-density lipoprotein particle receptor activity [GO:0005041] (molecular function) Sources: GOC:bf, ISBN:0198506732 Relationships: is a type of lipoprotein particle receptor activity [GO:0030228]; has part low-density lipoprotein particle binding [GO:0030169] Definition: Combining with a low-density lipoprotein particle and delivering the low-density lipoprotein particle into the cell via endocytosis. Also known as: LDL receptor, LDLR activity, low-density lipoprotein receptor activity